{
  "term_label": "late endosome",
  "gene_symbol": "ELAPOR1",
  "gene_name": "Endosome_lysosome-associated apoptosis and autophagy regulator 1",
  "gene": "UniProtKB:Q6UXG2",
  "term_id": "GO:0005770"
}